{
  "gene_name": "T cell receptor delta joining 3 (Fragment)",
  "gene": "UniProtKB:A0A075B6W1",
  "term_id": "UNKNOWN:0003",
  "gene_symbol": "TRDJ3",
  "term_label": "Unknown cellular component"
}